tryptophan dehydrogenase activity [GO:0050363] (molecular function) Definition: Catalysis of the reaction: L-tryptophan + NAD(P)+ = (indol-3-yl)pyruvate + NH3 + NAD(P)H + H+. Also known as: L-Trp-dehydrogenase activity, L-tryptophan dehydrogenase activity, L-tryptophan:NAD(P)+ oxidoreductase (deaminating), NAD(P)+-L-tryptophan dehydrogenase activity, TDH, TrpDH activity Sources: EC:1.4.1.19, MetaCyc:TRYPTOPHAN-DEHYDROGENASE-RXN Relationships: is a type of oxidoreductase activity, acting on the CH-NH2 group of donors, NAD or NADP as acceptor [GO:0016639]